{
  "gene_symbol": "INCENP",
  "gene": "UniProtKB:Q9NQS7",
  "term_id": "GO:1990385",
  "gene_name": "Inner centromere protein",
  "term_label": "meiotic spindle midzone"
}